{
  "gene_name": "Stearoyl-CoA desaturase 5",
  "gene": "UniProtKB:Q86SK9",
  "gene_symbol": "SCD5",
  "term_label": "iron ion binding",
  "term_id": "GO:0005506"
}